{
  "gene": "UniProtKB:Q8NDZ0",
  "term_label": "Unknown molecular function",
  "gene_symbol": "BEND2",
  "term_id": "UNKNOWN:0001",
  "gene_name": "BEN domain-containing protein 2"
}